{
  "gene_symbol": "SYT11",
  "term_id": "GO:0017158",
  "gene": "UniProtKB:Q9BT88",
  "gene_name": "Synaptotagmin-11",
  "term_label": "regulation of calcium ion-dependent exocytosis"
}